{
  "gene_symbol": "FBRSL1",
  "gene_name": "Fibrosin-1-like protein",
  "gene": "UniProtKB:Q9HCM7",
  "term_id": "UNKNOWN:0002",
  "term_label": "Unknown biological process"
}